response to cytokinesis checkpoint signaling [GO:0072399] (BP) Also known as: cytokinesis checkpoint effector process, response to signal involved in cytokinesis checkpoint Definition: A process that occurs in response to signals generated as a result of cytokinesis checkpoint signaling. Relationships: is a type of response to cell cycle checkpoint signaling [GO:0072396] Sources: GOC:mtg_cell_cycle Regulation: regulated by regulation of response to cytokinesis checkpoint signaling [GO:1902147]; positively regulated by GO:1902148